{
  "term_label": "nuclear import signal receptor activity",
  "gene": "UniProtKB:Q14974",
  "gene_name": "Importin subunit beta-1",
  "term_id": "GO:0061608",
  "gene_symbol": "KPNB1"
}